{
  "gene": "UniProtKB:Q9Y3Q3",
  "term_label": "Golgi organization",
  "gene_name": "Transmembrane emp24 domain-containing protein 3",
  "term_id": "GO:0007030",
  "gene_symbol": "TMED3"
}